{
  "term_label": "membrane",
  "gene": "UniProtKB:Q9GZU3",
  "term_id": "GO:0016020",
  "gene_name": "Transmembrane protein 39B",
  "gene_symbol": "TMEM39B"
}